{
  "gene_symbol": "MTFP1",
  "gene": "UniProtKB:Q9UDX5",
  "term_id": "GO:0005739",
  "term_label": "mitochondrion",
  "gene_name": "Mitochondrial fission process protein 1"
}